{
  "gene_name": "Putative uncharacterized protein BRD3OS",
  "gene_symbol": "BRD3OS",
  "term_id": "UNKNOWN:0001",
  "term_label": "Unknown molecular function",
  "gene": "UniProtKB:A0A1B0GUI7"
}